neurofibrillary tangle [GO:0097418] (cellular component) Note: Neurofibrillary tangles have been found in aging population; their formation is increased in Alzheimer's disease patients (and in other neurological diseases) compared to normal controls (see PMID:848276 and PMID:8584267). Sources: NIF_Subcellular:nlx_subcell_20090201, NIF_Subcellular:nlx_subcell_20090202, NIF_Subcellular:sao2409833926 Also known as: flame-shaped neurofibrillary tangle, star-shaped neurofibrillary tangle Relationships: is a type of GO:0016234 Definition: Intracellular mass of paired, helically wound protein filaments (also called PHF) lying in the cytoplasm of neuronal cell bodies and neuritic cell processes. Neurofibrillary tangles contain an abnormally phosphorylated form of a microtubule-associated protein, tau. The shape of these inclusions may resemble a flame or a star.